{
  "gene": "UniProtKB:Q8WXI7",
  "term_label": "Unknown molecular function",
  "gene_name": "Mucin-16",
  "gene_symbol": "MUC16",
  "term_id": "UNKNOWN:0001"
}